{
  "gene_symbol": "SNAPC3",
  "gene": "UniProtKB:Q92966",
  "term_id": "GO:0001006",
  "term_label": "RNA polymerase III type 3 promoter sequence-specific DNA binding",
  "gene_name": "snRNA-activating protein complex subunit 3"
}